{
  "term_id": "GO:0005759",
  "gene": "UniProtKB:O95822",
  "term_label": "mitochondrial matrix",
  "gene_name": "Malonyl-CoA decarboxylase, mitochondrial",
  "gene_symbol": "MLYCD"
}